{
  "gene": "UniProtKB:O95388",
  "gene_name": "CCN family member 4",
  "term_id": "GO:0008201",
  "gene_symbol": "CCN4",
  "term_label": "heparin binding"
}